{
  "gene_name": "Iron-sulfur cluster co-chaperone protein HscB",
  "gene_symbol": "HSCB",
  "term_label": "mitochondrion",
  "term_id": "GO:0005739",
  "gene": "UniProtKB:Q8IWL3"
}